{
  "gene_name": "E3 ubiquitin-protein ligase Midline-1",
  "gene": "UniProtKB:O15344",
  "term_id": "UNKNOWN:0001",
  "term_label": "Unknown molecular function",
  "gene_symbol": "MID1"
}